{
  "gene_name": "Syntaxin-10",
  "term_label": "SNARE binding",
  "gene": "UniProtKB:O60499",
  "term_id": "GO:0000149",
  "gene_symbol": "STX10"
}